{
  "gene_symbol": "WWC3",
  "term_id": "GO:0046621",
  "gene": "UniProtKB:Q9ULE0",
  "gene_name": "Protein WWC3",
  "term_label": "negative regulation of organ growth"
}